{
  "gene_symbol": "HLA-DRA",
  "gene_name": "HLA class II histocompatibility antigen, DR alpha chain",
  "term_label": "MHC class II protein complex binding",
  "gene": "UniProtKB:P01903",
  "term_id": "GO:0023026"
}